intracellular monoatomic cation homeostasis [GO:0030003] (biological process) Definition: A homeostatic process involved in the maintenance of a steady state level of monoatomic cations within a cell. Monatomic cations (also called simple cations) are cations consisting of exactly one atom. Relationships: is a type of intracellular monoatomic ion homeostasis [GO:0006873]; is a type of monoatomic cation homeostasis [GO:0055080] Sources: GOC:ceb, GOC:mah Also known as: cellular cation homeostasis, cellular monoatomic cation homeostasis Subtypes: intracellular calcium ion homeostasis [GO:0006874], intracellular cobalt ion homeostasis [GO:0006877], GO:0006878, intracellular iron ion homeostasis [GO:0006879], intracellular zinc ion homeostasis [GO:0006882], intracellular sodium ion homeostasis [GO:0006883], intracellular magnesium ion homeostasis [GO:0010961], intracellular potassium ion homeostasis [GO:0030007], intracellular manganese ion homeostasis [GO:0030026], regulation of cellular pH [GO:0030641], GO:0035785